{
  "gene": "UniProtKB:Q4VX76",
  "gene_name": "Synaptotagmin-like protein 3",
  "term_id": "GO:0070382",
  "term_label": "exocytic vesicle",
  "gene_symbol": "SYTL3"
}